{
  "term_label": "broad specificity oxidative DNA demethylase activity",
  "gene_symbol": "ALKBH1",
  "term_id": "GO:0035516",
  "gene": "UniProtKB:Q13686",
  "gene_name": "Nucleic acid dioxygenase ALKBH1"
}